chondrocyte proliferation [GO:0035988] (biological process) Relationships: is a type of cell population proliferation [GO:0008283] Also known as: cartilage cell proliferation, chondrocyte cell proliferation References: PMID:21484705 Sources: CL:0000138, GOC:yaf Definition: The multiplication or reproduction of chondrocytes by cell division, resulting in the expansion of their population. A chondrocyte is a polymorphic cell that forms cartilage. Regulation: negatively regulated by GO:1902731; positively regulated by positive regulation of chondrocyte proliferation [GO:1902732]